{
  "term_id": "GO:0050910",
  "gene": "UniProtKB:Q8TDI7",
  "term_label": "detection of mechanical stimulus involved in sensory perception of sound",
  "gene_symbol": "TMC2",
  "gene_name": "Transmembrane channel-like protein 2"
}